{
  "term_id": "GO:0030550",
  "term_label": "acetylcholine receptor inhibitor activity",
  "gene": "UniProtKB:P0DP58",
  "gene_symbol": "LYNX1",
  "gene_name": "Ly-6_neurotoxin-like protein 1"
}